{
  "term_id": "UNKNOWN:0003",
  "gene_name": "SH3KBP1-binding protein 1",
  "term_label": "Unknown cellular component",
  "gene_symbol": "SHKBP1",
  "gene": "UniProtKB:Q8TBC3"
}